response to corticotropin-releasing hormone [GO:0043435] (biological process) Also known as: response to CRF stimulus, response to CRH stimulus, response to corticoliberin stimulus, response to corticotropin-releasing factor stimulus, response to corticotropin-releasing hormone stimulus Relationships: is a type of response to peptide hormone [GO:0043434] Subtypes: GO:0071376 Definition: Any process that results in a change in state or activity of a cell or an organism (in terms of movement, secretion, enzyme production, gene expression, etc.) as a result of a corticotropin-releasing hormone stimulus. Corticotropin-releasing hormone is a peptide hormone involved in the stress response. References: PMID:11027914, PMID:15134857 Sources: Wikipedia:Corticotropin-releasing_hormone